{
  "gene": "UniProtKB:A0A0J9YX35",
  "gene_name": "Immunoglobulin heavy variable 3-64D",
  "term_label": "immunoglobulin mediated immune response",
  "gene_symbol": "IGHV3-64D",
  "term_id": "GO:0016064"
}